{
  "gene": "UniProtKB:P51504",
  "term_label": "regulation of transcription by RNA polymerase II",
  "term_id": "GO:0006357",
  "gene_name": "Zinc finger protein 80",
  "gene_symbol": "ZNF80"
}